{
  "gene_symbol": "FDXR",
  "term_label": "steroid biosynthetic process",
  "term_id": "GO:0006694",
  "gene": "UniProtKB:P22570",
  "gene_name": "NADPH:adrenodoxin oxidoreductase, mitochondrial"
}